ketogluconate catabolic process [GO:0046181] (biological process) Sources: ISBN:0198506732 Definition: The chemical reactions and pathways resulting in the breakdown of ketogluconate, the anion of ketogluconic acid, an aldonic acid derived from glucose containing a ketonic carbonyl group. Also known as: ketogluconate breakdown, ketogluconate catabolism, ketogluconate degradation Subtypes: GO:0019524 Relationships: is a type of aldonic acid catabolic process [GO:0046176]